{
  "term_label": "nucleus",
  "term_id": "GO:0005634",
  "gene": "UniProtKB:A6NNF4",
  "gene_symbol": "ZNF726",
  "gene_name": "Zinc finger protein 726"
}